lymphocyte mediated immunity [GO:0002449] (biological process) Relationships: is a type of leukocyte mediated immunity [GO:0002443] Subtypes: GO:0002228, T cell mediated immunity [GO:0002456], B cell mediated immunity [GO:0019724] Sources: GOC:add, GO_REF:0000022, ISBN:0781735149 Regulation: regulated by regulation of lymphocyte mediated immunity [GO:0002706]; negatively regulated by negative regulation of lymphocyte mediated immunity [GO:0002707]; positively regulated by GO:0002708 Also known as: cell-mediated immunity, cellular immune response Definition: Any process involved in the carrying out of an immune response by a lymphocyte.